{
  "gene_name": "GA-binding protein subunit beta-1",
  "gene_symbol": "GABPB1",
  "term_id": "GO:0045944",
  "gene": "UniProtKB:Q06547",
  "term_label": "positive regulation of transcription by RNA polymerase II"
}